regulation of cell proliferation involved in kidney development [GO:1901722] (biological process) Subtypes: regulation of glomerular mesangial cell proliferation [GO:0072124], GO:0090095, negative regulation of cell proliferation involved in kidney development [GO:1901723], positive regulation of cell proliferation involved in kidney development [GO:1901724], regulation of cell proliferation involved in mesonephros development [GO:2000606] Relationships: is a type of regulation of cell population proliferation [GO:0042127]; regulates cell proliferation involved in kidney development [GO:0072111] References: PMID:18182616 Sources: GOC:TermGenie Definition: Any process that modulates the frequency, rate or extent of cell proliferation involved in kidney development.